regulation of chemokine activity [GO:1900136] (biological process) Definition: Any process that modulates the frequency, rate or extent of chemokine activity. Sources: GOC:TermGenie Relationships: is a type of regulation of cytokine activity [GO:0060300]; regulates chemokine activity [GO:0008009] Subtypes: negative regulation of chemokine activity [GO:1900137]